aerobic respiration, using sulfur or sulfate as electron donor [GO:0019414] (biological process) Also known as: aerobic respiration, using sulphur or sulphate as electron donor Definition: An aerobic respiration process in which a sulfur-containing molecule (hydrogen sulfide, sulfur, sulfite, thiosulfate, and various polythionates) is oxidized. References: PMID:11425697 Relationships: is a type of GO:0009060; is a type of energy derivation by oxidation of reduced inorganic compounds [GO:0015975]